negative regulation of mammary gland involution [GO:1903520] (biological process) Also known as: down regulation of mammary gland involution, down-regulation of mammary gland involution, downregulation of mammary gland involution, inhibition of mammary gland involution References: PMID:23164222 Sources: GOC:TermGenie, GOC:dph, GO_REF:0000058 Relationships: is a type of negative regulation of tissue remodeling [GO:0034104]; is a type of regulation of mammary gland involution [GO:1903519]; negatively regulates mammary gland involution [GO:0060056] Definition: Any process that stops, prevents or reduces the frequency, rate or extent of mammary gland involution.